{
  "term_label": "Unknown molecular function",
  "gene": "UniProtKB:Q9BVK8",
  "term_id": "UNKNOWN:0001",
  "gene_name": "BOS complex subunit TMEM147",
  "gene_symbol": "TMEM147"
}